{
  "gene_name": "AP-2 complex subunit mu",
  "term_label": "AP-2 adaptor complex",
  "gene": "UniProtKB:Q96CW1",
  "gene_symbol": "AP2M1",
  "term_id": "GO:0030122"
}